long-term synaptic potentiation [GO:0060291] (BP) Also known as: long-term potentiation, LTP Definition: A process that modulates synaptic plasticity such that synapses are changed resulting in the increase in the rate, or frequency of synaptic transmission at the synapse. Sources: GOC:dgh, GOC:dph Relationships: is a type of regulation of synaptic plasticity [GO:0048167]; is a type of positive regulation of synaptic transmission [GO:0050806] Regulation: regulated by GO:1900271; negatively regulated by negative regulation of long-term synaptic potentiation [GO:1900272]; positively regulated by positive regulation of long-term synaptic potentiation [GO:1900273]